ergot alkaloid biosynthetic process [GO:0035837] (biological process) Also known as: ergot alkaloid anabolism, ergot alkaloid biosynthesis, ergot alkaloid formation, ergot alkaloid synthesis Subtypes: GO:1900569, fumigaclavine C biosynthetic process [GO:1900809] Relationships: is a type of terpenoid indole alkaloid biosynthetic process [GO:0009709] Regulation: regulated by regulation of ergot alkaloid biosynthetic process [GO:1900822]; negatively regulated by GO:1900823; positively regulated by positive regulation of ergot alkaloid biosynthetic process [GO:1900824] Sources: GOC:yaf Definition: The chemical reactions and pathways resulting in the formation of an ergot alkaloid.